negative regulation of uterine smooth muscle relaxation [GO:1900720] (biological process) Relationships: is a type of regulation of uterine smooth muscle relaxation [GO:1900719]; is_a negative regulation of relaxation of smooth muscle [GO:1901081]; RO_0002212 uterine smooth muscle relaxation [GO:0044558] Also known as: down regulation of smooth muscle relaxation of the uterus, down regulation of uterine smooth muscle relaxation, down-regulation of smooth muscle relaxation of the uterus, down-regulation of uterine smooth muscle relaxation, downregulation of smooth muscle relaxation of the uterus, downregulation of uterine smooth muscle relaxation, inhibition of smooth muscle relaxation of the uterus, negative regulation of smooth muscle relaxation of the uterus, inhibition of uterine smooth muscle relaxation Sources: GOC:TermGenie Definition: Any process that stops, prevents or reduces the frequency, rate or extent of uterine smooth muscle relaxation.